{
  "gene_name": "Protein sel-1 homolog 2",
  "term_label": "ERAD pathway",
  "term_id": "GO:0036503",
  "gene_symbol": "SEL1L2",
  "gene": "UniProtKB:Q5TEA6"
}